{
  "gene": "UniProtKB:Q9NS00",
  "term_label": "Unknown cellular component",
  "term_id": "UNKNOWN:0003",
  "gene_symbol": "C1GALT1",
  "gene_name": "Glycoprotein-N-acetylgalactosamine 3-beta-galactosyltransferase 1"
}